tolerance induction in Peyer's patch [GO:0002389] (biological process) Definition: Tolerance induction taking place in the Peyer's patches. Sources: GOC:jal, ISBN:0781735149 Relationships: is a type of immune response in Peyer's patch [GO:0002388]; is a type of tolerance induction in gut-associated lymphoid tissue [GO:0002394]